{
  "term_id": "GO:0007346",
  "gene": "UniProtKB:Q9NVM9",
  "gene_name": "Integrator complex subunit 13",
  "gene_symbol": "INTS13",
  "term_label": "regulation of mitotic cell cycle"
}